{
  "gene": "UniProtKB:Q8WVM7",
  "gene_name": "Cohesin subunit SA-1",
  "gene_symbol": "STAG1",
  "term_label": "cohesin complex",
  "term_id": "GO:0008278"
}